positive regulation of chemokine production [GO:0032722] (biological process) Also known as: up regulation of chemokine production, up-regulation of chemokine production, upregulation of chemokine production, activation of chemokine production, positive regulation of chemokine biosynthetic process, positive regulation of chemokine secretion, stimulation of chemokine production Sources: GOC:mah Definition: Any process that activates or increases the frequency, rate, or extent of chemokine production. Subtypes: positive regulation of fractalkine production [GO:0032724], GO:0035396, positive regulation of chemokine (C-C motif) ligand 6 production [GO:0035533], positive regulation of monocyte chemotactic protein-1 production [GO:0071639], positive regulation of macrophage inflammatory protein 1 alpha production [GO:0071642], positive regulation of chemokine (C-C motif) ligand 4 production [GO:0071645], positive regulation of macrophage inflammatory protein-1 gamma production [GO:0071648], positive regulation of chemokine (C-C motif) ligand 5 production [GO:0071651], positive regulation of chemokine (C-C motif) ligand 1 production [GO:0071654], GO:0071660, positive regulation of chemokine (C-C motif) ligand 20 production [GO:1903886], GO:2000340, positive regulation of chemokine (C-X-C motif) ligand 2 production [GO:2000343] Relationships: is a type of positive regulation of cytokine production [GO:0001819]; is a type of regulation of chemokine production [GO:0032642]; positively regulates chemokine production [GO:0032602]